catenin-TCF7L2 complex [GO:0071664] (cellular component) References: PMID:14661054 Sources: GOC:BHF, GOC:rl, GOC:vk Also known as: catenin-TCF4 complex Relationships: is a type of nuclear protein-containing complex [GO:0140513] Subtypes: beta-catenin-TCF7L2 complex [GO:0070369], GO:0071665 Definition: A protein complex that contains a catenin and TCF7L2 (TCF4), binds to the TCF DNA motif within a promoter element, and is involved in the regulation of WNT target gene transcription.